{
  "gene_symbol": "OTX1",
  "gene_name": "Homeobox protein OTX1",
  "term_label": "midbrain development",
  "gene": "UniProtKB:P32242",
  "term_id": "GO:0030901"
}